{
  "gene": "UniProtKB:P62136",
  "gene_name": "Serine_threonine-protein phosphatase PP1-alpha catalytic subunit",
  "term_label": "cytoplasm",
  "gene_symbol": "PPP1CA",
  "term_id": "GO:0005737"
}